{
  "term_label": "heat shock protein binding",
  "term_id": "GO:0031072",
  "gene_symbol": "HSPA1B",
  "gene": "UniProtKB:P0DMV9",
  "gene_name": "Heat shock 70 kDa protein 1B"
}